{
  "term_label": "phosphatidylcholine lysophospholipase activity",
  "gene_symbol": "ABHD4",
  "gene_name": "(Lyso)-N-acylphosphatidylethanolamine lipase",
  "gene": "UniProtKB:Q8TB40",
  "term_id": "GO:0004622"
}